Slit-Robo signaling complex [GO:0071666] (cellular component) References: PMID:17062560, PMID:18359766 Sources: GOC:sart Relationships: is a type of protein-carbohydrate complex [GO:0032992] Also known as: Slit-Robo signalling complex Definition: A protein-carbohydrate complex that consists of a transmembrane roundabout (Robo) receptor, an extracellular Slit ligand and heparin/heparan sulfate.